{
  "term_label": "positive regulation of enamel mineralization",
  "gene": "UniProtKB:Q17RF5",
  "term_id": "GO:0070175",
  "gene_name": "Odontogenesis associated phosphoprotein",
  "gene_symbol": "ODAPH"
}